membrane depolarization during AV node cell action potential [GO:0086045] (biological process) Also known as: membrane depolarization during AV node cardiac muscle cell action potential, membrane depolarization during atrioventricular node cardiac muscle cell action potential Regulation: regulated by regulation of membrane depolarization during AV node cell action potential [GO:1905027]; negatively regulated by GO:1905028; positively regulated by positive regulation of membrane depolarization during AV node cell action potential [GO:1905029] Definition: The process in which AV node cardiac muscle cell membrane potential changes in the depolarizing direction from the negative resting potential towards the positive membrane potential that will be the peak of the action potential. Relationships: is a type of membrane depolarization during cardiac muscle cell action potential [GO:0086012]; is part of AV node cell action potential [GO:0086016] Sources: GOC:BHF, GOC:mtg_cardiac_conduct_nov11